molybdopterin molybdotransferase activity [GO:0061599] (molecular function) Definition: Catalysis of the reaction adenylyl-molybdopterin + molybdate = molybdenum cofactor + AMP. Sources: EC:2.10.1.1, GOC:dph Relationships: is a type of transferase activity [GO:0016740]